{
  "term_label": "neurotransmitter receptor activity",
  "gene_symbol": "HTR2A",
  "gene_name": "5-hydroxytryptamine receptor 2A",
  "term_id": "GO:0030594",
  "gene": "UniProtKB:P28223"
}